{
  "gene": "UniProtKB:Q8NBS9",
  "gene_name": "Thioredoxin domain-containing protein 5",
  "gene_symbol": "TXNDC5",
  "term_label": "protein folding",
  "term_id": "GO:0006457"
}